{
  "gene_symbol": "AUP1",
  "term_id": "UNKNOWN:0001",
  "gene_name": "Lipid droplet-regulating VLDL assembly factor AUP1",
  "gene": "UniProtKB:Q9Y679",
  "term_label": "Unknown molecular function"
}